{
  "term_label": "cytoplasm",
  "term_id": "GO:0005737",
  "gene_name": "UBX domain-containing protein 6",
  "gene_symbol": "UBXN6",
  "gene": "UniProtKB:Q9BZV1"
}